{
  "term_label": "negative regulation of gene expression",
  "gene": "UniProtKB:Q53GL7",
  "gene_name": "Protein mono-ADP-ribosyltransferase PARP10",
  "gene_symbol": "PARP10",
  "term_id": "GO:0010629"
}